symbiont-mediated suppression of host cytoplasmic pattern recognition receptor signaling pathway via inhibition of TBK1 activity [GO:0039723] (biological process) Definition: Any process in which a symbiont stops, prevents, or reduces a cytoplasmic pattern recognition receptor signaling pathway in a host organism by reducing the activity of a host serine/threonine kinase TBK1. References: PMID:22171259, PMID:34084167 Note: This term is for annotation of symbiont proteins that counteract the host anti-microbial innate immune response. Relationships: is a type of symbiont-mediated suppression of cytoplasmic pattern recognition receptor signaling pathway [GO:0039537] Also known as: suppression by virus of host viral-induced cytoplasmic pattern recognition receptor signaling pathway via inhibition of TBK1 activity, inhibition of host TBK1 by virus, suppression by virus of host TBK1 activity, symbiont-mediated suppression of host TKB signaling